{
  "gene_name": "Sorbin and SH3 domain-containing protein 2",
  "term_id": "GO:0030425",
  "gene_symbol": "SORBS2",
  "term_label": "dendrite",
  "gene": "UniProtKB:O94875"
}